{
  "term_label": "Unknown biological process",
  "gene_symbol": "EMC7",
  "term_id": "UNKNOWN:0002",
  "gene": "UniProtKB:Q9NPA0",
  "gene_name": "ER membrane protein complex subunit 7"
}